{
  "gene_symbol": "UBE2R2",
  "term_id": "GO:0000209",
  "gene_name": "Ubiquitin-conjugating enzyme E2 R2",
  "gene": "UniProtKB:Q712K3",
  "term_label": "protein polyubiquitination"
}